T cell tolerance induction in mucosal-associated lymphoid tissue [GO:0002403] (biological process) Relationships: is a type of tolerance induction in mucosal-associated lymphoid tissue [GO:0002401]; is_a peripheral T cell tolerance induction [GO:0002458] Definition: Tolerance induction taking place in the mucosal-associated lymphoid tissue (MALT) mediated by T cells. References: PMID:16551263 Sources: GOC:jal, ISBN:0781735149 Also known as: T cell tolerance induction in MALT